{
  "term_id": "GO:0005634",
  "term_label": "nucleus",
  "gene_symbol": "PARN",
  "gene_name": "Poly(A)-specific ribonuclease PARN",
  "gene": "UniProtKB:O95453"
}